{
  "gene_name": "Sperm-egg fusion protein TMEM95",
  "gene_symbol": "TMEM95",
  "term_id": "GO:0007342",
  "term_label": "fusion of sperm to egg plasma membrane involved in single fertilization",
  "gene": "UniProtKB:Q3KNT9"
}